{
  "gene": "UniProtKB:Q6NYC1",
  "gene_symbol": "JMJD6",
  "term_label": "phagocytosis",
  "gene_name": "Bifunctional arginine demethylase and lysyl-hydroxylase JMJD6",
  "term_id": "GO:0006909"
}